{
  "gene": "UniProtKB:Q9NRI5",
  "gene_name": "Disrupted in schizophrenia 1 protein",
  "gene_symbol": "DISC1",
  "term_label": "postsynaptic density",
  "term_id": "GO:0014069"
}